{
  "gene_name": "Putative protein FAM90A15P",
  "term_id": "UNKNOWN:0003",
  "gene_symbol": "FAM90A15P",
  "term_label": "Unknown cellular component",
  "gene": "UniProtKB:P0C7V4"
}